cellobiose epimerase activity [GO:0047736] (molecular function) Definition: Catalysis of the reaction: cellobiose = D-glucosyl-D-mannose. Relationships: is_a racemase and epimerase activity, acting on carbohydrates and derivatives [GO:0016857] Also known as: cellobiose 2-epimerase activity Sources: EC:5.1.3.11, MetaCyc:CELLOBIOSE-EPIMERASE-RXN